{
  "gene_name": "Proteasome subunit beta type-1",
  "gene": "UniProtKB:P20618",
  "gene_symbol": "PSMB1",
  "term_id": "GO:0005839",
  "term_label": "proteasome core complex"
}